{
  "gene_symbol": "SLC26A4",
  "gene_name": "Pendrin",
  "gene": "UniProtKB:O43511",
  "term_label": "sulfate transmembrane transporter activity",
  "term_id": "GO:0015116"
}